{
  "gene_name": "Phosphatidylinositol 4-kinase type 2-beta",
  "gene": "UniProtKB:Q8TCG2",
  "gene_symbol": "PI4K2B",
  "term_id": "GO:0007030",
  "term_label": "Golgi organization"
}